{
  "term_id": "GO:0004674",
  "gene_symbol": "RIOK3",
  "term_label": "protein serine/threonine kinase activity",
  "gene": "UniProtKB:O14730",
  "gene_name": "Serine_threonine-protein kinase RIO3"
}